{
  "term_id": "UNKNOWN:0003",
  "gene_name": "Putative transcript Y 12 protein",
  "gene_symbol": "TTTY12",
  "term_label": "Unknown cellular component",
  "gene": "UniProtKB:Q9BZ98"
}